phosphatidylcholine biosynthesis from phosphatidylethanolamine [GO:0090638] (biological process) Definition: The phosphatidylcholine biosynthetic process that depends on direct conversion of the phosphatidyl-base phosphatidylethanolamine to phosphatidylcholine by successive methylations. Sources: MetaCyc:PWY-6825 Relationships: is a type of GO:0006656